exocytic vesicle membrane [GO:0099501] (cellular component) Sources: GOC:dos Also known as: secretory vesicle membrane Relationships: is a type of transport vesicle membrane [GO:0030658]; is part of GO:0070382 Subtypes: synaptic vesicle membrane [GO:0030672] Definition: The lipid bilayer surrounding an exocytic vesicle.